{
  "term_label": "cytoplasm",
  "gene_name": "Differentially expressed in FDCP 6 homolog",
  "gene_symbol": "DEF6",
  "gene": "UniProtKB:Q9H4E7",
  "term_id": "GO:0005737"
}